{
  "term_id": "GO:0016746",
  "term_label": "acyltransferase activity",
  "gene_name": "Lysophospholipid acyltransferase 2",
  "gene": "UniProtKB:Q6ZWT7",
  "gene_symbol": "MBOAT2"
}